{
  "gene": "UniProtKB:P36406",
  "term_label": "GTP binding",
  "term_id": "GO:0005525",
  "gene_symbol": "TRIM23",
  "gene_name": "E3 ubiquitin-protein ligase TRIM23"
}